{
  "term_label": "brain development",
  "gene_name": "Ataxin-1",
  "term_id": "GO:0007420",
  "gene_symbol": "ATXN1",
  "gene": "UniProtKB:P54253"
}